{
  "gene_name": "Keratin, type I cytoskeletal 16",
  "term_id": "GO:0045109",
  "term_label": "intermediate filament organization",
  "gene": "UniProtKB:P08779",
  "gene_symbol": "KRT16"
}